CHOP-C/EBP complex [GO:0036488] (cellular component) Definition: A heterodimeric protein complex that is composed of the transcription factor CHOP (GADD153) and a member of the C/EBP family of transcription factors. References: PMID:1547942 Sources: GOC:PARL, GOC:bf Also known as: CHOP-C/EBP dimer, CHOP-C/EBP heterodimer, GADD153-C/EBP complex, GADD153-C/EBP-alpha complex Relationships: is a type of RNA polymerase II transcription regulator complex [GO:0090575]